myosin phosphatase complex [GO:0017023] (cellular component) Definition: An enzyme complex that catalyzes the removal of the phosphate group from phosphomyosin. Composed of a PP1 catalytic subunit (PP1c/PPP1CB) and a myosin phosphatase targeting subunit (MYPT1/PPP1R12A). Relationships: is a type of protein serine/threonine phosphatase complex [GO:0008287] References: PMID:30076859